{
  "gene_name": "Nuclear nucleic acid-binding protein C1D",
  "term_id": "GO:0000460",
  "gene_symbol": "C1D",
  "term_label": "maturation of 5.8S rRNA",
  "gene": "UniProtKB:Q13901"
}